{
  "gene": "UniProtKB:P43626",
  "gene_name": "Killer cell immunoglobulin-like receptor 2DL1",
  "gene_symbol": "KIR2DL1",
  "term_id": "GO:0140375",
  "term_label": "immune receptor activity"
}